{
  "gene_symbol": "TEDDM1",
  "gene": "UniProtKB:Q5T9Z0",
  "term_label": "Unknown biological process",
  "gene_name": "Transmembrane epididymal protein 1",
  "term_id": "UNKNOWN:0002"
}